{
  "gene_name": "Phosphoglucomutase-like protein 5",
  "gene_symbol": "PGM5",
  "gene": "UniProtKB:Q15124",
  "term_id": "GO:0005975",
  "term_label": "carbohydrate metabolic process"
}